{
  "gene_symbol": "GABRB3",
  "term_label": "synaptic transmission, GABAergic",
  "gene_name": "Gamma-aminobutyric acid receptor subunit beta-3",
  "gene": "UniProtKB:P28472",
  "term_id": "GO:0051932"
}